{
  "gene_symbol": "WWC1",
  "gene_name": "Protein KIBRA",
  "term_id": "GO:0005737",
  "gene": "UniProtKB:Q8IX03",
  "term_label": "cytoplasm"
}